{
  "gene_name": "Putative uncharacterized protein encoded by LINC01465",
  "term_id": "UNKNOWN:0002",
  "gene": "UniProtKB:Q8N7H1",
  "term_label": "Unknown biological process",
  "gene_symbol": "LINC01465"
}